protein localization to site of double-strand break [GO:1990166] (biological process) Also known as: protein localisation to site of double-strand break, protein localization to double-strand break site, protein localization to site of DSB Definition: Any process in which a protein is transported to, or maintained at, a region of a chromosome at which a DNA double-strand break has occurred. References: PMID:23080121 Sources: GOC:mah Relationships: is a type of protein localization to chromosome [GO:0034502]